{
  "term_id": "GO:0015630",
  "gene_name": "Tubulin monoglycylase TTLL3",
  "gene": "UniProtKB:Q9Y4R7",
  "term_label": "microtubule cytoskeleton",
  "gene_symbol": "TTLL3"
}